{
  "term_id": "UNKNOWN:0002",
  "gene_name": "Trafficking protein particle complex subunit 9",
  "gene": "UniProtKB:Q96Q05",
  "term_label": "Unknown biological process",
  "gene_symbol": "TRAPPC9"
}